{
  "term_label": "Unknown molecular function",
  "gene": "UniProtKB:Q9P127",
  "term_id": "UNKNOWN:0001",
  "gene_name": "Leucine zipper protein 4",
  "gene_symbol": "LUZP4"
}